{
  "term_label": "cytoplasm",
  "term_id": "GO:0005737",
  "gene_name": "PABIR family member 2",
  "gene_symbol": "PABIR2",
  "gene": "UniProtKB:Q7Z309"
}